{
  "gene": "UniProtKB:Q8IXP5",
  "gene_symbol": "POU2AF2",
  "term_label": "Unknown biological process",
  "gene_name": "POU domain class 2-associating factor 2",
  "term_id": "UNKNOWN:0002"
}